{
  "gene_symbol": "PHETA1",
  "term_id": "GO:0042147",
  "gene": "UniProtKB:Q8N4B1",
  "term_label": "retrograde transport, endosome to Golgi",
  "gene_name": "Sesquipedalian-1"
}